{
  "term_label": "midbody",
  "gene": "UniProtKB:M0R2J8",
  "term_id": "GO:0030496",
  "gene_name": "Doublecortin domain-containing protein 1",
  "gene_symbol": "DCDC1"
}